{
  "gene_name": "Cyclin-D1-binding protein 1",
  "term_id": "GO:0005634",
  "term_label": "nucleus",
  "gene_symbol": "CCNDBP1",
  "gene": "UniProtKB:O95273"
}